{
  "gene_symbol": "MUSTN1",
  "term_label": "Unknown cellular component",
  "gene": "UniProtKB:Q8IVN3",
  "gene_name": "Musculoskeletal embryonic nuclear protein 1",
  "term_id": "UNKNOWN:0003"
}